{
  "gene": "UniProtKB:P19474",
  "gene_name": "E3 ubiquitin-protein ligase TRIM21",
  "term_label": "cytoplasm",
  "gene_symbol": "TRIM21",
  "term_id": "GO:0005737"
}